{
  "term_id": "GO:0005886",
  "term_label": "plasma membrane",
  "gene_symbol": "ADAM30",
  "gene_name": "Disintegrin and metalloproteinase domain-containing protein 30",
  "gene": "UniProtKB:Q9UKF2"
}